{
  "term_id": "GO:0005248",
  "gene_symbol": "PKD2",
  "gene_name": "Polycystin-2",
  "term_label": "voltage-gated sodium channel activity",
  "gene": "UniProtKB:Q13563"
}